{
  "gene_name": "UV excision repair protein RAD23 homolog A",
  "term_label": "proteasome binding",
  "gene_symbol": "RAD23A",
  "term_id": "GO:0070628",
  "gene": "UniProtKB:P54725"
}